{
  "term_label": "cytoplasm",
  "gene_name": "Ran-binding protein 10",
  "gene": "UniProtKB:Q6VN20",
  "gene_symbol": "RANBP10",
  "term_id": "GO:0005737"
}